{
  "term_label": "eye development",
  "gene_name": "Putative homeobox protein Meis3-like 1",
  "gene_symbol": "MEIS3P1",
  "term_id": "GO:0001654",
  "gene": "UniProtKB:A6NDR6"
}